{
  "gene": "UniProtKB:Q7RTY3",
  "gene_name": "Putative serine protease 45",
  "term_label": "extracellular space",
  "gene_symbol": "PRSS45P",
  "term_id": "GO:0005615"
}